farnesol 2-isomerase activity [GO:0047885] (MF) Relationships: is a type of cis-trans isomerase activity [GO:0016859] Sources: EC:5.2.1.9, RHEA:13401 Also known as: 2-trans,6-trans-farnesol 2-cis-trans-isomerase activity, farnesol isomerase activity Definition: Catalysis of the reaction: 2-trans,6-trans-farnesol = 2-cis,6-trans-farnesol.